{
  "gene_symbol": "CIRBP-AS1",
  "gene_name": "Putative uncharacterized protein CIRBP-AS1",
  "term_label": "Unknown molecular function",
  "term_id": "UNKNOWN:0001",
  "gene": "UniProtKB:Q8TBR5"
}